{
  "gene_symbol": "SRP14",
  "term_id": "UNKNOWN:0001",
  "gene": "UniProtKB:P37108",
  "term_label": "Unknown molecular function",
  "gene_name": "Signal recognition particle 14 kDa protein"
}